{
  "gene": "UniProtKB:Q8WW22",
  "term_label": "cytosol",
  "gene_name": "DnaJ homolog subfamily A member 4",
  "gene_symbol": "DNAJA4",
  "term_id": "GO:0005829"
}